{
  "gene": "UniProtKB:P59025",
  "term_id": "GO:0006612",
  "gene_symbol": "RTP1",
  "gene_name": "Receptor-transporting protein 1",
  "term_label": "protein targeting to membrane"
}